{
  "gene_symbol": "KCTD14",
  "gene": "UniProtKB:Q9BQ13",
  "term_label": "Unknown biological process",
  "gene_name": "BTB_POZ domain-containing protein KCTD14",
  "term_id": "UNKNOWN:0002"
}